{
  "term_id": "GO:0005739",
  "gene": "UniProtKB:P30405",
  "gene_symbol": "PPIF",
  "gene_name": "Peptidyl-prolyl cis-trans isomerase F, mitochondrial",
  "term_label": "mitochondrion"
}